aminoglycoside 6'-N-acetyltransferase activity [GO:0047663] (MF) Sources: EC:2.3.1.82, RHEA:16449 Definition: Catalysis of the reaction: acetyl-CoA + kanamycin B = N(6')-acetylkanamycin B + CoA + H+. This is acetylation of the 6'-amino group of the 6-deoxy-6-aminoglucose ring. Also known as: aminoglycoside N6'-acetyltransferase activity, acetyl-CoA:kanamycin-B N6'-acetyltransferase activity, kanamycin 6'-N-acetyltransferase activity, 6'-aminoglycoside-N-acetyltransferase activity, AAC(6') activity, aminoglycoside-6'-acetyltransferase activity, aminoglycoside-6-N-acetyltransferase activity Relationships: is a type of GO:0034069